{
  "gene_symbol": "MASTL",
  "term_label": "protein serine/threonine kinase activity",
  "gene_name": "Serine_threonine-protein kinase greatwall",
  "term_id": "GO:0004674",
  "gene": "UniProtKB:Q96GX5"
}